{
  "term_id": "GO:1902711",
  "gene": "UniProtKB:P31644",
  "gene_name": "Gamma-aminobutyric acid receptor subunit alpha-5",
  "term_label": "GABA-A receptor complex",
  "gene_symbol": "GABRA5"
}